{
  "term_label": "cell division site",
  "gene": "UniProtKB:Q8IYM1",
  "gene_name": "Septin-12",
  "gene_symbol": "SEPTIN12",
  "term_id": "GO:0032153"
}